{
  "gene_name": "Astacin-like metalloendopeptidase",
  "term_id": "GO:0004222",
  "gene": "UniProtKB:Q6HA08",
  "gene_symbol": "ASTL",
  "term_label": "metalloendopeptidase activity"
}